{
  "gene_symbol": "PGLYRP1",
  "gene_name": "Peptidoglycan recognition protein 1",
  "term_id": "GO:0005615",
  "gene": "UniProtKB:O75594",
  "term_label": "extracellular space"
}